protein-lipid-RNA complex [GO:1990684] (cellular component) Subtypes: HDL-containing protein-lipid-RNA complex [GO:1990685], LDL-containing protein-lipid-RNA complex [GO:1990686] Also known as: miRNA-lipoprotein complex References: PMID:21423178, PMID:22028337, PMID:23559634 Sources: GOC:vesicles Relationships: is a type of protein-containing complex [GO:0032991] Note: Examples of protein-lipid-RNA complexes are described in PMID:21423178 and PMID:23559634, both showing evidence that high-density lipoprotein (HDL) and, to a lesser extent, low-density lipoprotein (HDL) transport endogenous microRNAs (miRNAs) and deliver them to recipient cells with functional targeting capabilities. Also see fig. 1 in the review PMID:22028337. Not to be confused with GO:0034364 'high-density lipoprotein particle' or GO:0034362 'low-density lipoprotein particle', which describe complexes of proteins and lipids only, without RNAs. Definition: A macromolecular complex containing separate protein, lipid and RNA molecules. Separate in this context means not covalently bound to each other.